regulation of apical ectodermal ridge formation [GO:1905140] (biological process) Relationships: is a type of GO:0022603; RO_0002211 apical ectodermal ridge formation [GO:1905139] Definition: Any process that modulates the frequency, rate or extent of apical ectodermal ridge formation. References: PMID:18359901 Sources: GOC:TermGenie, GO_REF:0000058 Subtypes: negative regulation of apical ectodermal ridge formation [GO:1905141], positive regulation of apical ectodermal ridge formation [GO:1905142] Also known as: regulation of apical epidermal ridge formation, regulation of AER formation, regulation of crista ectodermalis apicalis formation